{
  "term_id": "GO:0030160",
  "term_label": "synaptic receptor adaptor activity",
  "gene_name": "SH3 and multiple ankyrin repeat domains protein 2",
  "gene_symbol": "SHANK2",
  "gene": "UniProtKB:Q9UPX8"
}